{
  "gene_name": "Soluble scavenger receptor cysteine-rich domain-containing protein SSC5D",
  "gene": "UniProtKB:A1L4H1",
  "term_label": "extracellular space",
  "term_id": "GO:0005615",
  "gene_symbol": "SSC5D"
}